negative regulation of actin filament depolymerization [GO:0030835] (biological process) Sources: GOC:mah Subtypes: actin filament capping [GO:0051693] Definition: Any process that stops, prevents, or reduces the frequency, rate or extent of actin depolymerization. Note: Note that this term was split from 'negative regulation of actin polymerization and/or depolymerization ; GO:0045757' (sibling term 'negative regulation of actin polymerization ; GO:0030837'). Relationships: is a type of regulation of actin filament depolymerization [GO:0030834]; is a type of GO:0051494; is_a GO:1901880; is a type of GO:1902904; negatively regulates actin filament depolymerization [GO:0030042] Also known as: negative regulation of actin polymerization and/or depolymerization, actin filament stabilization, down regulation of actin filament depolymerization, down-regulation of actin filament depolymerization, downregulation of actin filament depolymerization, negative regulation of actin depolymerization, inhibition of actin filament depolymerization